{
  "gene_name": "Spermatogenesis-associated serine-rich protein 2",
  "term_id": "UNKNOWN:0001",
  "gene_symbol": "SPATS2",
  "gene": "UniProtKB:Q86XZ4",
  "term_label": "Unknown molecular function"
}